{
  "term_label": "siRNA binding",
  "term_id": "GO:0035197",
  "gene_name": "Putative protein FAM172B",
  "gene_symbol": "ARB2BP",
  "gene": "UniProtKB:A6NC97"
}